beta-arrestin-dependent dopamine receptor signaling pathway [GO:0160213] (BP) Definition: A beta-arrestin-dependent signaling pathway initiated by a dopamine binding to its receptor on the surface of a target cell, and ending with the regulation of a downstream cellular process. References: PMID:21711983, PMID:25671228 Relationships: is a type of cell surface receptor signaling pathway [GO:0007166]; is part of GO:1903351